{
  "gene_name": "Proline-rich protein 23C",
  "gene_symbol": "PRR23C",
  "gene": "UniProtKB:Q6ZRP0",
  "term_id": "UNKNOWN:0003",
  "term_label": "Unknown cellular component"
}